response to desipramine [GO:1904307] (biological process) Subtypes: GO:1904308 Relationships: is a type of response to nitrogen compound [GO:1901698] Definition: Any process that results in a change in state or activity of a cell or an organism (in terms of movement, secretion, enzyme production, gene expression, etc.) as a result of a desipramine stimulus. References: PMID:20549303 Sources: GOC:TermGenie, GO_REF:0000071